{
  "gene_name": "E3 ubiquitin-protein ligase RNF166",
  "gene_symbol": "RNF166",
  "term_id": "GO:0006511",
  "gene": "UniProtKB:Q96A37",
  "term_label": "ubiquitin-dependent protein catabolic process"
}